superoxide-generating NADH oxidase activity [GO:0106291] (molecular function) Sources: RHEA:63184 Definition: Catalysis of the reaction: NADH + 2 O2 = H+ + NAD+ + 2 superoxide. Relationships: is a type of superoxide-generating NAD(P)H oxidase activity [GO:0016175]